{
  "term_label": "negative regulation of DNA-templated transcription",
  "term_id": "GO:0045892",
  "gene_name": "Sterile alpha motif domain-containing protein 7",
  "gene": "UniProtKB:Q7Z3H4",
  "gene_symbol": "SAMD7"
}